{
  "term_id": "GO:0032190",
  "gene_name": "Zona pellucida sperm-binding protein 4",
  "gene": "UniProtKB:Q12836",
  "term_label": "acrosin binding",
  "gene_symbol": "ZP4"
}